{
  "gene_symbol": "ZDHHC3",
  "gene": "UniProtKB:Q9NYG2",
  "term_label": "protein localization to plasma membrane",
  "gene_name": "Palmitoyltransferase ZDHHC3",
  "term_id": "GO:0072659"
}